{
  "term_label": "fibroblast growth factor receptor signaling pathway",
  "term_id": "GO:0008543",
  "gene_name": "Fibroblast growth factor 18",
  "gene": "UniProtKB:O76093",
  "gene_symbol": "FGF18"
}